negative regulation of maintenance of bipolar cell polarity regulating cell shape [GO:0061362] (biological process) Definition: Any process that decreases the frequency, rate or extent of maintenance of bipolar cell polarity regulating cell shape. Sources: GOC:dph Relationships: is a type of GO:2000115; is a type of negative regulation of establishment or maintenance of bipolar cell polarity regulating cell shape [GO:2000750]; negatively regulates maintenance of bipolar cell polarity regulating cell shape [GO:0061305]